{
  "term_label": "Unknown biological process",
  "term_id": "UNKNOWN:0002",
  "gene_symbol": "NQO1",
  "gene_name": "NAD(P)H dehydrogenase [quinone] 1",
  "gene": "UniProtKB:P15559"
}